{
  "gene": "UniProtKB:P15407",
  "term_label": "nucleus",
  "gene_symbol": "FOSL1",
  "gene_name": "Fos-related antigen 1",
  "term_id": "GO:0005634"
}